aerobic respiration, using ferrous ions as electron donor [GO:0019411] (biological process) Definition: The metabolic process in which ferrous ions (Fe2+) are oxidized to ferric ions (Fe3+) to generate energy, coupled to the reduction of carbon dioxide. Sources: ISBN:3131084111 Relationships: is a type of aerobic respiration [GO:0009060]; is a type of energy derivation by oxidation of reduced inorganic compounds [GO:0015975]